{
  "gene_name": "Thymidylate synthase",
  "gene": "UniProtKB:P04818",
  "term_label": "dTMP biosynthetic process",
  "gene_symbol": "TYMS",
  "term_id": "GO:0006231"
}